{
  "term_label": "prostaglandin biosynthetic process",
  "gene_symbol": "PTGIS",
  "term_id": "GO:0001516",
  "gene": "UniProtKB:Q16647",
  "gene_name": "Prostacyclin synthase"
}